{
  "gene_name": "Glucosidase 2 subunit beta",
  "term_id": "GO:0006491",
  "gene": "UniProtKB:P14314",
  "gene_symbol": "PRKCSH",
  "term_label": "N-glycan processing"
}